{
  "gene_symbol": "NIPSNAP2",
  "term_id": "UNKNOWN:0001",
  "gene_name": "Protein NipSnap homolog 2",
  "term_label": "Unknown molecular function",
  "gene": "UniProtKB:O75323"
}